{
  "gene": "UniProtKB:Q14315",
  "gene_symbol": "FLNC",
  "gene_name": "Filamin-C",
  "term_label": "Unknown cellular component",
  "term_id": "UNKNOWN:0003"
}